{
  "gene_name": "ADP-ribosylation factor-like protein 13B",
  "gene_symbol": "ARL13B",
  "term_id": "GO:0060170",
  "gene": "UniProtKB:Q3SXY8",
  "term_label": "ciliary membrane"
}